{
  "gene": "UniProtKB:Q14160",
  "term_id": "GO:0043113",
  "gene_symbol": "SCRIB",
  "term_label": "receptor clustering",
  "gene_name": "Protein scribble homolog"
}